{
  "gene": "UniProtKB:P08912",
  "gene_symbol": "CHRM5",
  "term_label": "synapse",
  "term_id": "GO:0045202",
  "gene_name": "Muscarinic acetylcholine receptor M5"
}